{
  "term_id": "GO:0005737",
  "term_label": "cytoplasm",
  "gene_symbol": "GAMT",
  "gene_name": "Guanidinoacetate N-methyltransferase",
  "gene": "UniProtKB:Q14353"
}